{
  "term_label": "3-chloroallyl aldehyde dehydrogenase activity",
  "gene_name": "Aldehyde dehydrogenase, dimeric NADP-preferring",
  "gene_symbol": "ALDH3A1",
  "gene": "UniProtKB:P30838",
  "term_id": "GO:0004028"
}